{
  "term_id": "GO:0000460",
  "gene_name": "Exosome RNA helicase MTR4",
  "term_label": "maturation of 5.8S rRNA",
  "gene_symbol": "MTREX",
  "gene": "UniProtKB:P42285"
}